{
  "gene_symbol": "ABCA1",
  "term_id": "GO:0090556",
  "term_label": "phosphatidylserine floppase activity",
  "gene": "UniProtKB:O95477",
  "gene_name": "Phospholipid-transporting ATPase ABCA1"
}